{
  "gene_name": "Putative uncharacterized protein FLJ40140",
  "gene_symbol": "Q8N814",
  "gene": "UniProtKB:Q8N814",
  "term_id": "UNKNOWN:0003",
  "term_label": "Unknown cellular component"
}